{
  "gene": "UniProtKB:P11498",
  "gene_symbol": "PC",
  "gene_name": "Pyruvate carboxylase, mitochondrial",
  "term_label": "pyruvate carboxylase activity",
  "term_id": "GO:0004736"
}